{
  "gene_name": "Succinate-semialdehyde dehydrogenase, mitochondrial",
  "gene_symbol": "ALDH5A1",
  "term_label": "mitochondrion",
  "gene": "UniProtKB:P51649",
  "term_id": "GO:0005739"
}